positive regulation of defense response to oomycetes [GO:1902290] (biological process) Definition: Any process that activates or increases the frequency, rate or extent of defense response to oomycetes. Relationships: is_a positive regulation of response to biotic stimulus [GO:0002833]; is_a positive regulation of defense response [GO:0031349]; is a type of positive regulation of response to external stimulus [GO:0032103]; is a type of regulation of defense response to oomycetes [GO:1902288]; positively regulates defense response to oomycetes [GO:0002229] References: PMID:16040633 Sources: GOC:TermGenie Also known as: up regulation of defense response to oomycetes, up-regulation of defense response to oomycetes, upregulation of defense response to oomycetes, activation of defense response to oomycetes